{
  "term_label": "nucleus",
  "gene_symbol": "BOLA2",
  "gene": "UniProtKB:Q9H3K6",
  "gene_name": "BolA-like protein 2",
  "term_id": "GO:0005634"
}